{
  "term_id": "GO:0007186",
  "gene_symbol": "OR5AK2",
  "gene_name": "Olfactory receptor 5AK2",
  "term_label": "G protein-coupled receptor signaling pathway",
  "gene": "UniProtKB:Q8NH90"
}